{
  "gene": "UniProtKB:Q96PQ0",
  "gene_name": "VPS10 domain-containing receptor SorCS2",
  "term_label": "Unknown biological process",
  "gene_symbol": "SORCS2",
  "term_id": "UNKNOWN:0002"
}